{
  "gene_name": "G-protein coupled receptor 87",
  "term_label": "Unknown cellular component",
  "term_id": "UNKNOWN:0003",
  "gene_symbol": "GPR87",
  "gene": "UniProtKB:Q9BY21"
}